{
  "term_label": "nucleus",
  "gene_symbol": "TMEM250",
  "gene_name": "Transmembrane protein 250",
  "gene": "UniProtKB:H0YL14",
  "term_id": "GO:0005634"
}